{
  "term_label": "Unknown biological process",
  "gene": "UniProtKB:P54849",
  "gene_name": "Epithelial membrane protein 1",
  "term_id": "UNKNOWN:0002",
  "gene_symbol": "EMP1"
}